{
  "gene": "UniProtKB:Q01432",
  "gene_name": "AMP deaminase 3",
  "gene_symbol": "AMPD3",
  "term_label": "IMP biosynthetic process",
  "term_id": "GO:0006188"
}